{
  "gene_symbol": "SSU72L1",
  "gene_name": "RNA polymerase II subunit A C-terminal domain phosphatase SSU72 like protein 1",
  "gene": "UniProtKB:A0A1W2PQ27",
  "term_id": "GO:0008420",
  "term_label": "RNA polymerase II CTD heptapeptide repeat phosphatase activity"
}